{
  "gene_name": "Partitioning defective 6 homolog beta",
  "gene_symbol": "PARD6B",
  "term_label": "establishment or maintenance of cell polarity",
  "term_id": "GO:0007163",
  "gene": "UniProtKB:Q9BYG5"
}